{
  "gene_name": "Melanoma-associated antigen D1",
  "term_id": "GO:0000122",
  "gene_symbol": "MAGED1",
  "gene": "UniProtKB:Q9Y5V3",
  "term_label": "negative regulation of transcription by RNA polymerase II"
}